transmembrane transport from lysosomal lumen to cytosol [GO:0170063] (biological process) Relationships: is a type of lysosomal transport [GO:0007041]; is a type of vacuolar transmembrane transport [GO:0034486] References: PMID:26631267 Subtypes: GO:0141204, L-lysine transmembrane transport from lysosomal lumen to cytosol [GO:1904916], GO:1904917, L-histidine transmembrane transport from lysosomal lumen to cytosol [GO:1904918], GO:1904919 Definition: The directed movement of a solute from the lysosomal lumen across the lysosomal membrane and into the cytosol.